{
  "term_label": "L-leucine binding",
  "gene_name": "Sestrin-3",
  "gene": "UniProtKB:P58005",
  "gene_symbol": "SESN3",
  "term_id": "GO:0070728"
}